{
  "term_label": "Unknown molecular function",
  "term_id": "UNKNOWN:0001",
  "gene": "UniProtKB:Q6PID8",
  "gene_name": "Kelch domain-containing protein 10",
  "gene_symbol": "KLHDC10"
}